response to dinitrophenol [GO:1904641] (biological process) Also known as: response to dinitrophenols References: PMID:24336883 Sources: GOC:TermGenie, GO_REF:0000071 Definition: Any process that results in a change in state or activity of a cell or an organism (in terms of movement, secretion, enzyme production, gene expression, etc.) as a result of a dinitrophenol stimulus. Relationships: is a type of response to nitrogen compound [GO:1901698]; is a type of response to oxygen-containing compound [GO:1901700] Subtypes: GO:1904642